response to isolation stress [GO:0035900] (biological process) References: PMID:20203532 Sources: GOC:bf Relationships: is_a response to stress [GO:0006950] Also known as: response to social isolation Definition: Any process that results in a change in state or activity of a cell or an organism (in terms of movement, secretion, enzyme production, gene expression, etc.) as a result of a lack of contact with other members of the same species. Subtypes: cellular response to isolation stress [GO:0035901]